{
  "gene": "UniProtKB:P23588",
  "gene_name": "Eukaryotic translation initiation factor 4B",
  "term_id": "GO:0003723",
  "gene_symbol": "EIF4B",
  "term_label": "RNA binding"
}